{
  "gene_name": "Inhibitor of growth protein 4",
  "gene": "UniProtKB:Q9UNL4",
  "term_label": "nucleus",
  "term_id": "GO:0005634",
  "gene_symbol": "ING4"
}